{
  "term_id": "GO:0000981",
  "gene_symbol": "ZNF621",
  "term_label": "DNA-binding transcription factor activity, RNA polymerase II-specific",
  "gene_name": "Zinc finger protein 621",
  "gene": "UniProtKB:Q6ZSS3"
}